{
  "gene_name": "Protein SHQ1 homolog",
  "gene_symbol": "SHQ1",
  "gene": "UniProtKB:Q6PI26",
  "term_id": "GO:0005654",
  "term_label": "nucleoplasm"
}